{
  "term_id": "GO:0005923",
  "gene_name": "Claudin-8",
  "gene": "UniProtKB:P56748",
  "term_label": "bicellular tight junction",
  "gene_symbol": "CLDN8"
}